{
  "term_id": "GO:0007005",
  "gene": "UniProtKB:Q96TA2",
  "gene_symbol": "YME1L1",
  "term_label": "mitochondrion organization",
  "gene_name": "ATP-dependent zinc metalloprotease YME1L1"
}